trehalase activity [GO:0015927] (molecular function) Definition: Catalysis of the hydrolysis of trehalose or a trehalose derivative. References: PMID:31925485 Sources: GOC:ai Relationships: is a type of GO:0004553 Subtypes: alpha,alpha-trehalase activity [GO:0004555], alpha,alpha-phosphotrehalase activity [GO:0008788]